{
  "gene_name": "Homeobox protein Hox-A9",
  "gene_symbol": "HOXA9",
  "term_id": "GO:0003700",
  "term_label": "DNA-binding transcription factor activity",
  "gene": "UniProtKB:P31269"
}